regulation of presynaptic dense core granule exocytosis [GO:0099161] (biological process) References: PMID:17881523 Sources: GOC:dos Also known as: regulation of presynaptic dense core vesicle exocytosis Definition: Any process that modulates the frequency, rate or extent of presynaptic dense core granule exocytosis. Relationships: is_a GO:0099171; is a type of regulation of calcium ion-dependent exocytosis of neurotransmitter [GO:1903233]; is a type of regulation of dense core granule exocytosis [GO:1905413]; regulates presynaptic dense core vesicle exocytosis [GO:0099525]